{
  "term_id": "UNKNOWN:0002",
  "gene_name": "MORC family CW-type zinc finger protein 4",
  "gene": "UniProtKB:Q8TE76",
  "term_label": "Unknown biological process",
  "gene_symbol": "MORC4"
}